{
  "term_label": "Unknown cellular component",
  "term_id": "UNKNOWN:0003",
  "gene_name": "Ubiquitin-associated domain-containing protein 2",
  "gene_symbol": "UBAC2",
  "gene": "UniProtKB:Q8NBM4"
}